{
  "gene": "UniProtKB:P24462",
  "term_id": "GO:0070989",
  "gene_symbol": "CYP3A7",
  "gene_name": "Cytochrome P450 3A7",
  "term_label": "oxidative demethylation"
}